{
  "term_label": "Unknown molecular function",
  "gene_name": "ATP synthase-coupling factor 6, mitochondrial",
  "gene_symbol": "ATP5PF",
  "gene": "UniProtKB:P18859",
  "term_id": "UNKNOWN:0001"
}